inorganic ion import across plasma membrane [GO:0099587] (BP) Definition: The directed movement of inorganic ions from outside of a cell, across the plasma membrane and into the cytosol. Subtypes: inorganic anion import across plasma membrane [GO:0098658], inorganic cation import across plasma membrane [GO:0098659] Also known as: inorganic ion import into cell Relationships: is a type of GO:0098739 Sources: GOC:dos